{
  "gene_name": "Olfactory receptor 11G2",
  "term_label": "Unknown biological process",
  "gene": "UniProtKB:Q8NGC1",
  "term_id": "UNKNOWN:0002",
  "gene_symbol": "OR11G2"
}